{
  "gene_symbol": "HOOK2",
  "gene": "UniProtKB:Q96ED9",
  "term_id": "GO:0005737",
  "term_label": "cytoplasm",
  "gene_name": "Protein Hook homolog 2"
}